{
  "gene": "UniProtKB:P14923",
  "gene_name": "Junction plakoglobin",
  "gene_symbol": "JUP",
  "term_id": "GO:0005912",
  "term_label": "adherens junction"
}